positive regulation of sterol import [GO:2000911] (biological process) Definition: Any process that activates or increases the frequency, rate or extent of sterol import. Sources: GOC:obol Also known as: positive regulation of sterol influx, positive regulation of sterol uptake Relationships: is a type of positive regulation of sterol transport [GO:0032373]; is a type of regulation of sterol import [GO:2000909]; positively regulates sterol import [GO:0035376]